{
  "term_label": "DNA endonuclease activity",
  "term_id": "GO:0004520",
  "gene": "UniProtKB:Q5FWF4",
  "gene_symbol": "ZRANB3",
  "gene_name": "DNA annealing helicase and endonuclease ZRANB3"
}